{
  "term_label": "Unknown molecular function",
  "gene": "UniProtKB:Q7Z628",
  "gene_name": "Neuroepithelial cell-transforming gene 1 protein",
  "term_id": "UNKNOWN:0001",
  "gene_symbol": "NET1"
}